cytidine catabolic process [GO:0006216] (biological process) Definition: The chemical reactions and pathways resulting in the breakdown of cytidine, cytosine riboside, a widely distributed nucleoside. Sources: GOC:ai Also known as: cytidine breakdown, cytidine catabolism, cytidine degradation Relationships: is a type of cytidine metabolic process [GO:0046087]; is a type of GO:0046133